glycoprotein 3-alpha-L-fucosyltransferase activity [GO:0018392] (molecular function) Sources: EC:2.4.1.214, RHEA:24444 Also known as: GDP-L-fucose:asparagine-linked N-acetylglucosamine alpha(1,3)-fucosyltransferase activity, GDP-L-Fuc:Asn-linked GlcNAc alpha-1,3-fucosyltransferase activity, GDP-L-Fuc:Asn-linked GlcNAc alpha1,3-fucosyltransferase activity, GDP-L-Fuc:N-acetyl-beta-D-glucosaminide alpha-1,3-fucosyltransferase activity, GDP-L-Fuc:N-acetyl-beta-D-glucosaminide alpha1,3-fucosyltransferase activity, GDP-L-fucose:glycoprotein (L-fucose to asparagine-linked N-acetylglucosamine of 4-N-{N-acetyl-beta-D-glucosaminyl-(1->2)-alpha-D-mannosyl-(1->3)-[N-acetyl-beta-D-glucosaminyl-(1->2)-alpha-D-mannosyl-(1->6)]-beta-D-mannosyl-(1->4)-N-acetyl-beta-D-glucosaminyl-(1->4)-N-acetyl-beta-D-glucosaminyl}asparagine) 3-alpha-L-fucosyl-transferase activity, GDP-L-fucose:glycoprotein (L-fucose to asparagine-linked N-acetylglucosamine of N4-{N-acetyl-beta-D-glucosaminyl-(1->2)-alpha-D-mannosyl-(1->3)-[N-acetyl-beta-D-glucosaminyl-(1->2)-alpha-D-mannosyl-(1->6)]-beta-D-mannosyl-(1->4)-N-acetyl-beta-D-glucosaminyl-(1->4)-N-acetyl-beta-D-glucosaminyl}asparagine) 3-alpha-L-fucosyl-transferase activity, GDP-fucose:beta-N-acetylglucosamine (Fuc to (Fuc-alpha-1->6-GlcNAc)-Asn-peptide) alpha-1->3-fucosyltransferase activity, GDP-fucose:beta-N-acetylglucosamine (Fuc to (Fucalpha1->6-GlcNAc)-Asn-peptide) alpha1->3-fucosyltransferase activity, GDP-fucose:beta-N-acetylglucosamine (Fuc to (Fucalpha1->6GlcNAc)-Asn-peptide) alpha1->3-fucosyltransferase activity Definition: Catalysis of the reaction: N(4)-{N-acetyl-beta-D-glucosaminyl-(1->2)-alpha-D-mannosyl-(1->3)-[N-acetyl-beta-D-glucosaminyl-(1->2)-alpha-D-mannosyl-(1->6)]-beta-D-mannosyl-(1->4)-N-acetyl-beta-D-glucosaminyl-(1->4)-N-acetyl-beta-D-glucosaminyl}-L-asparagine + GDP-L-fucose = N(4)-{N-acetyl-beta-D-glucosaminyl-(1->2)-alpha-D-mannosyl-(1->3)-[N-acetyl-beta-D-glucosaminyl-(1->2)-alpha-D-mannosyl-(1->6)]-beta-D-mannosyl-(1->4)-N-acetyl-beta-D-glucosaminyl-(1->4)-[alpha-L-fucosyl-(1->3)]-N-acetyl-beta-D-glucosaminyl}-L-asparagine + GDP + H+. Relationships: is a type of alpha-(1->3)-fucosyltransferase activity [GO:0046920]; is a type of GO:0140103